regulation of basement membrane assembly involved in embryonic body morphogenesis [GO:1904259] (biological process) Relationships: is a type of GO:0045995; is a type of regulation of basement membrane organization [GO:0110011]; is a type of regulation of extracellular matrix assembly [GO:1901201]; RO_0002211 basement membrane assembly involved in embryonic body morphogenesis [GO:2001197] Subtypes: GO:1904260, positive regulation of basement membrane assembly involved in embryonic body morphogenesis [GO:1904261] Definition: Any process that modulates the frequency, rate or extent of basement membrane assembly involved in embryonic body morphogenesis. References: PMID:23940118 Sources: GOC:TermGenie, GOC:als, GO_REF:0000058